{
  "gene_symbol": "HBG2",
  "gene_name": "Hemoglobin subunit gamma-2",
  "term_label": "hemoglobin alpha binding",
  "gene": "UniProtKB:P69892",
  "term_id": "GO:0031721"
}